{
  "term_id": "GO:0070273",
  "term_label": "phosphatidylinositol-4-phosphate binding",
  "gene": "UniProtKB:P57764",
  "gene_symbol": "GSDMD",
  "gene_name": "Gasdermin-D"
}